{
  "term_id": "GO:0030198",
  "term_label": "extracellular matrix organization",
  "gene": "UniProtKB:Q3B7J2",
  "gene_symbol": "GFOD2",
  "gene_name": "Glucose-fructose oxidoreductase domain-containing protein 2"
}